aspartic-type endopeptidase inhibitor activity [GO:0019828] (molecular function) Also known as: aspartic protease inhibitor activity Sources: GOC:ai Definition: Binds to and stops, prevents or reduces the activity of aspartic-type endopeptidases. Relationships: is a type of GO:0004866; negatively regulates aspartic-type endopeptidase activity [GO:0004190]